{
  "gene_symbol": "A4GNT",
  "gene_name": "Alpha-1,4-N-acetylglucosaminyltransferase",
  "term_label": "Unknown cellular component",
  "term_id": "UNKNOWN:0003",
  "gene": "UniProtKB:Q9UNA3"
}